CROP complex [GO:0170071] (cellular component) References: PMID:35466426 Definition: A complex involved in membrane fission during protein exchange in endo-lysosomal compartments. CROP joins members of two protein families: the peripheral subunits of retromer, a coat forming endosomal transport carriers, and membrane inserting PROPPINs. Also known as: Cutting Retromer-On-PROPPIN Relationships: is a type of GO:0032991